{
  "gene_name": "Fibrocystin-L",
  "gene": "UniProtKB:Q86WI1",
  "term_id": "UNKNOWN:0001",
  "term_label": "Unknown molecular function",
  "gene_symbol": "PKHD1L1"
}